{
  "gene_symbol": "FETUB",
  "term_id": "GO:0008191",
  "gene_name": "Fetuin-B",
  "term_label": "metalloendopeptidase inhibitor activity",
  "gene": "UniProtKB:Q9UGM5"
}